apicomplexan dense granule [GO:0020026] (cellular component) Relationships: is a type of GO:0030141 Definition: Electron-dense organelle with a granular internal matrix found in a apicomplexan parasite; contains proteins destined to be secreted into the parasitophorous vacuole following parasite invasion of a host cell. Also known as: dense body References: PMID:15978597, PMID:35302693 Sources: GOC:mb, GOC:mtg_sensu